{
  "gene_symbol": "BCL2L12",
  "term_id": "GO:0005634",
  "gene_name": "Bcl-2-like protein 12",
  "term_label": "nucleus",
  "gene": "UniProtKB:Q9HB09"
}